regulation of fungal-type cell wall biogenesis [GO:0032995] (biological process) Relationships: is a type of GO:0044087; is a type of regulation of cell wall organization or biogenesis [GO:1903338]; regulates fungal-type cell wall biogenesis [GO:0009272] Definition: Any process that modulates the process in which a cell wall is synthesized, aggregates, and bonds together. The fungal-type cell wall contains beta-glucan and may contain chitin. Subtypes: regulation of fungal-type cell wall (1->3)-alpha-glucan biosynthetic process [GO:0070610], GO:0090093 Sources: GOC:dph, GOC:mah, GOC:tb Also known as: regulation of chitin- and beta-glucan-containing cell wall biogenesis